{
  "gene_symbol": "TNNC1",
  "term_id": "GO:0048306",
  "term_label": "calcium-dependent protein binding",
  "gene": "UniProtKB:P63316",
  "gene_name": "Troponin C, slow skeletal and cardiac muscles"
}